N-acetylmuramic acid catabolic process [GO:0097173] (biological process) Definition: The chemical reactions and pathways resulting in the breakdown of N-acetylmuramic acid (MurNAc), a monosaccharide derivative of N-acetylglucosamine. Relationships: is a type of GO:0046395; is a type of N-acetylmuramic acid metabolic process [GO:0097172] Regulation: positively regulated by GO:0160159 Also known as: N-acetylmuramate breakdown, N-acetylmuramate catabolic process, N-acetylmuramate catabolism, N-acetylmuramate degradation, N-acetylmuramic acid breakdown, N-acetylmuramic acid catabolism, N-acetylmuramic acid degradation Sources: GOC:yaf